CCR11 chemokine receptor binding [GO:0031736] (molecular function) Sources: GOC:mah, GOC:nln Also known as: CCR11 chemokine receptor ligand Relationships: is a type of CCR chemokine receptor binding [GO:0048020] Definition: Binding to a CCR11 chemokine receptor.